{
  "gene_name": "Receptor-type tyrosine-protein phosphatase N2",
  "gene": "UniProtKB:Q92932",
  "term_label": "synapse",
  "term_id": "GO:0045202",
  "gene_symbol": "PTPRN2"
}